{
  "term_label": "phototransduction, visible light",
  "gene_symbol": "GNAT1",
  "term_id": "GO:0007603",
  "gene_name": "Guanine nucleotide-binding protein G(t) subunit alpha-1",
  "gene": "UniProtKB:P11488"
}